{
  "gene": "UniProtKB:Q8NCS4",
  "gene_name": "Transmembrane protein 35B",
  "gene_symbol": "TMEM35B",
  "term_label": "Unknown cellular component",
  "term_id": "UNKNOWN:0003"
}